flavin adenine dinucleotide biosynthetic process [GO:0072388] (biological process) Relationships: is a type of nucleotide biosynthetic process [GO:0009165]; is a type of flavin-containing compound biosynthetic process [GO:0042727]; is a type of flavin adenine dinucleotide metabolic process [GO:0072387] Subtypes: FAD biosynthetic process [GO:0006747] Also known as: FAD or FADH2 biosynthetic process, flavin adenine dinucleotide anabolism, flavin adenine dinucleotide biosynthesis, flavin adenine dinucleotide formation, flavin adenine dinucleotide synthesis Definition: The chemical reactions and pathways resulting in the formation of flavin adenine dinucleotide, which acts as a coenzyme or prosthetic group of various flavoprotein oxidoreductase enzymes. Sources: GOC:mah